1-phosphatidylinositol-3-phosphate 5-kinase activity [GO:0000285] (molecular function) Sources: EC:2.7.1.150, RHEA:13609 Also known as: phosphatidylinositol-3-phosphate 5-kinase activity, ATP:1-phosphatidyl-1D-myo-inositol-3-phosphate 5-phosphotransferase activity, phosphatidylinositol 3-phosphate 5-kinase activity, type III PIP kinase activity Definition: Catalysis of the reaction: a 1-phosphatidyl-1D-myo-inositol 3-phosphate + ATP = a 1-phosphatidyl-1D-myo-inositol 3,5-bisphosphate + ADP + H+. Relationships: is a type of phosphatidylinositol kinase activity [GO:0052742]